{
  "gene": "UniProtKB:O60729",
  "gene_name": "Dual specificity protein phosphatase CDC14B",
  "gene_symbol": "CDC14B",
  "term_label": "microtubule cytoskeleton organization",
  "term_id": "GO:0000226"
}